alpha4-beta1 integrin-CD82 complex [GO:0070521] (cellular component) Definition: A protein complex that consists of an alpha4-beta1 integrin complex bound to membrane protein CD82, a member of the tetraspan family. References: PMID:8757325 Relationships: is a type of GO:0098797